{
  "gene": "UniProtKB:P0CG42",
  "term_id": "UNKNOWN:0002",
  "term_label": "Unknown biological process",
  "gene_name": "Putative protein FAM157B",
  "gene_symbol": "FAM157B"
}